beta-alanyl-dopamine hydrolase activity [GO:0003832] (molecular function) Also known as: N-beta-alanyl-dopamine hydrolase activity, NBAD hydrolase activity References: PMID:16299587 Sources: RHEA:73467 Definition: Catalysis of the reaction: beta-alanyl-dopamine + H2O = dopamine + beta-alanine. Relationships: is a type of hydrolase activity, acting on carbon-nitrogen (but not peptide) bonds, in linear amides [GO:0016811]